{
  "gene": "UniProtKB:P47884",
  "term_id": "GO:0007165",
  "term_label": "signal transduction",
  "gene_name": "Olfactory receptor 1D4",
  "gene_symbol": "OR1D4"
}